{
  "gene_name": "Ankyrin repeat domain-containing protein 54",
  "gene": "UniProtKB:Q6NXT1",
  "term_id": "GO:0019887",
  "gene_symbol": "ANKRD54",
  "term_label": "protein kinase regulator activity"
}